has_broad_synonym [oboInOwl#hasBroadSynonym]